vitamin D catabolic process [GO:0042369] (biological process) Also known as: vitamin D breakdown, vitamin D catabolism, vitamin D degradation, calciferol catabolic process, calciferol catabolism, cholecalciferol biosynthesis, cholecalciferol biosynthetic process, ergocalciferol biosynthesis, ergocalciferol biosynthetic process Subtypes: vitamin D3 catabolic process [GO:1901754] Definition: The chemical reactions and pathways resulting in the breakdown of vitamin D, any of a group of related, fat-soluble compounds that are derived from delta-5,7 steroids and play a central role in calcium metabolism. Specific forms of vitamin D include calciferol (ergocalciferol; vitamin D2) and cholecalciferol (calciol; vitamin D3). Relationships: is a type of steroid catabolic process [GO:0006706]; is a type of vitamin D metabolic process [GO:0042359]; is a type of fat-soluble vitamin catabolic process [GO:0042363] Sources: GOC:mah, ISBN:0471331309